{
  "gene": "UniProtKB:Q8TC05",
  "gene_symbol": "MDM1",
  "term_label": "Unknown molecular function",
  "gene_name": "Nuclear protein MDM1",
  "term_id": "UNKNOWN:0001"
}